{
  "gene_symbol": "TLNRD1",
  "term_id": "UNKNOWN:0002",
  "gene_name": "Talin rod domain-containing protein 1",
  "term_label": "Unknown biological process",
  "gene": "UniProtKB:Q9H1K6"
}